{
  "term_id": "GO:0006633",
  "gene_name": "3-oxoacyl-[acyl-carrier-protein] synthase, mitochondrial",
  "gene_symbol": "OXSM",
  "term_label": "fatty acid biosynthetic process",
  "gene": "UniProtKB:Q9NWU1"
}